regulation of skeletal muscle fiber differentiation [GO:1902809] (biological process) Relationships: is a type of GO:0010830; is a type of regulation of skeletal muscle cell differentiation [GO:2001014]; regulates GO:0098528 Definition: Any process that modulates the frequency, rate or extent of skeletal muscle fiber differentiation. Subtypes: GO:1902810, positive regulation of skeletal muscle fiber differentiation [GO:1902811], regulation of tongue muscle cell differentiation [GO:2001035] References: PMID:17879321 Sources: GOC:TermGenie, GOC:mr, GO_REF:0000058